coniferin metabolic process [GO:0033491] (biological process) Sources: GOC:mah, MetaCyc:PWY-116 Also known as: coniferin metabolism Relationships: is a type of glycoside metabolic process [GO:0016137] Definition: The chemical reactions and pathways involving coniferin, 4-(3-hydroxyprop-1-en-1-yl)-2-methoxyphenyl beta-D-glucopyranoside.